prenyl-FMNH2 binding [GO:0120233] (molecular function) Also known as: prenylated FMNH2 binding Relationships: is a type of ribonucleotide binding [GO:0032553]; is a type of anion binding [GO:0043168] Definition: Binding to prenyl-FMNH2, a flavin mononucleotide obtained by prenylation of the N-10 position of FMNH2 followed by cyclisation. An essential cofactor for the decarboxylase enzymes UbiD and Fdc1. References: PMID:25647642, PMID:26083743, PMID:26083754 Sources: GOC:krc